{
  "term_label": "leukocyte cell-cell adhesion",
  "gene": "UniProtKB:Q86UX7",
  "term_id": "GO:0007159",
  "gene_symbol": "FERMT3",
  "gene_name": "Fermitin family homolog 3"
}